negative regulation of G protein-coupled receptor internalization [GO:1904021] (biological process) Definition: Any process that stops, prevents or reduces the frequency, rate or extent of G protein-coupled receptor internalization. Also known as: down regulation of G-protein coupled receptor internalization, down-regulation of G-protein coupled receptor internalization, downregulation of G-protein coupled receptor internalization, negative regulation of G-protein coupled receptor internalization, inhibition of G-protein coupled receptor internalization References: PMID:24732013 Sources: GOC:TermGenie, GO_REF:0000058 Relationships: is a type of GO:0002091; is a type of GO:1904020; negatively regulates G protein-coupled receptor internalization [GO:0002031]